{
  "gene": "UniProtKB:Q15185",
  "term_id": "GO:0005829",
  "gene_symbol": "PTGES3",
  "gene_name": "Prostaglandin E synthase 3",
  "term_label": "cytosol"
}